inositol phosphosphingolipid phospholipase activity [GO:0052712] (molecular function) Relationships: is a type of phospholipase C activity [GO:0004629] Sources: GOC:ai Subtypes: inositol phosphorylceramide phospholipase activity [GO:0052713] Definition: Catalysis of the reaction: inositol phosphosphingolipid + H2O = sphingolipid + phosphorylinositol.